{
  "gene": "UniProtKB:P18510",
  "gene_name": "Interleukin-1 receptor antagonist protein",
  "term_id": "GO:0005152",
  "term_label": "interleukin-1 receptor antagonist activity",
  "gene_symbol": "IL1RN"
}